{
  "gene": "UniProtKB:Q9NUV7",
  "term_id": "GO:0017059",
  "gene_name": "Serine palmitoyltransferase 3",
  "term_label": "serine palmitoyltransferase complex",
  "gene_symbol": "SPTLC3"
}